{
  "gene_symbol": "LEF1",
  "term_id": "GO:0006357",
  "term_label": "regulation of transcription by RNA polymerase II",
  "gene_name": "Lymphoid enhancer-binding factor 1",
  "gene": "UniProtKB:Q9UJU2"
}